{
  "term_id": "GO:0016460",
  "term_label": "myosin II complex",
  "gene_symbol": "MYL3",
  "gene_name": "Myosin light chain 3",
  "gene": "UniProtKB:P08590"
}